{
  "gene_symbol": "ZNF732",
  "term_label": "Unknown cellular component",
  "term_id": "UNKNOWN:0003",
  "gene": "UniProtKB:B4DXR9",
  "gene_name": "Zinc finger protein 732"
}